positive regulation of convergent extension involved in notochord morphogenesis [GO:1904138] (biological process) Also known as: up regulation of convergent extension involved in notochord morphogenesis, up-regulation of convergent extension involved in notochord morphogenesis, upregulation of convergent extension involved in notochord morphogenesis, activation of convergent extension involved in notochord morphogenesis Relationships: is a type of GO:1904105; is_a regulation of convergent extension involved in notochord morphogenesis [GO:1904136]; positively regulates convergent extension involved in notochord morphogenesis [GO:1904126] References: PMID:24892953 Sources: GOC:TermGenie, GOC:dph, GO_REF:0000058 Definition: Any process that activates or increases the frequency, rate or extent of convergent extension involved in notochord morphogenesis.